{
  "term_label": "Unknown molecular function",
  "gene": "UniProtKB:Q8WWQ2",
  "term_id": "UNKNOWN:0001",
  "gene_name": "Inactive heparanase-2",
  "gene_symbol": "HPSE2"
}